regulation of luteinizing hormone secretion [GO:0033684] (biological process) Definition: Any process that modulates the frequency, rate or extent of the regulated release of luteinizing hormone. Sources: GOC:mah Relationships: is a type of regulation of gonadotropin secretion [GO:0032276]; regulates luteinizing hormone secretion [GO:0032275] Subtypes: GO:0033685, positive regulation of luteinizing hormone secretion [GO:0033686]